{
  "gene_symbol": "CELSR3",
  "term_label": "axonogenesis",
  "gene": "UniProtKB:Q9NYQ7",
  "term_id": "GO:0007409",
  "gene_name": "Cadherin EGF LAG seven-pass G-type receptor 3"
}